{
  "gene_symbol": "TNNC1",
  "term_label": "skeletal muscle contraction",
  "gene": "UniProtKB:P63316",
  "gene_name": "Troponin C, slow skeletal and cardiac muscles",
  "term_id": "GO:0003009"
}